{
  "gene_name": "Transcription elongation factor A protein-like 8",
  "term_id": "UNKNOWN:0002",
  "gene_symbol": "TCEAL8",
  "gene": "UniProtKB:Q8IYN2",
  "term_label": "Unknown biological process"
}